{
  "gene": "UniProtKB:P36021",
  "gene_symbol": "SLC16A2",
  "term_label": "thyroid hormone transmembrane transporter activity",
  "gene_name": "Monocarboxylate transporter 8",
  "term_id": "GO:0015349"
}